{
  "term_id": "GO:0140227",
  "gene_symbol": "HTR3D",
  "term_label": "serotonin-gated cation-selective signaling pathway",
  "gene": "UniProtKB:Q70Z44",
  "gene_name": "5-hydroxytryptamine receptor 3D"
}